UDP-glucose transmembrane transporter activity [GO:0005460] (molecular function) Definition: Enables the transfer of a UDP-glucose from one side of a membrane to the other. UDP-glucose is a substance composed of glucose in glycosidic linkage with uridine diphosphate. Sources: GOC:ai, GOC:mtg_transport, ISBN:0815340729 Relationships: is a type of pyrimidine nucleotide-sugar transmembrane transporter activity [GO:0015165]; is part of UDP-glucose transmembrane transport [GO:0015786]